{
  "term_id": "UNKNOWN:0001",
  "term_label": "Unknown molecular function",
  "gene": "UniProtKB:Q5VZ46",
  "gene_symbol": "KIAA1614",
  "gene_name": "Uncharacterized protein KIAA1614"
}